positive regulation of cell integrity MAPK cascade [GO:1903139] (biological process) Definition: Any process that activates or increases the frequency, rate or extent of a cell integrity MAPK cascade. Sources: GOC:vw Also known as: positive regulation of MAPK cascade involved in cell wall organization or biogenesis, positive regulation of MAPKKK cascade involved in cell wall biogenesis, positive regulation of cell wal integrity MAPK pathway, positive regulation of cell wall biogenesis, MAPKKK cascade, activation of Mpk1 cascade, activation of PMK1-MAPK signal transduction pathway, activation of Pmk1 MAPK cell integrity signaling, activation of Pmk1 mitogen-activated protein kinase (MAPK) cell integrity pathway, activation of Slt2 cascade, activation of cell integrity MAPK pathway, positive regulation of Mpk1 cascade, positive regulation of PMK1-MAPK signal transduction pathway, positive regulation of Pmk1 MAPK cell integrity signaling, positive regulation of Pmk1 mitogen-activated protein kinase (MAPK) cell integrity pathway, positive regulation of Slt2 cascade Relationships: is a type of positive regulation of stress-activated MAPK cascade [GO:0032874]; is a type of regulation of cell integrity MAPK cascade [GO:1903137]; positively regulates GO:0000196